{
  "gene_symbol": "TSBP1",
  "gene_name": "Testis-expressed basic protein 1",
  "gene": "UniProtKB:Q5SRN2",
  "term_label": "Unknown molecular function",
  "term_id": "UNKNOWN:0001"
}